2-hydroxypropyl-CoM lyase activity [GO:0050555] (molecular function) Definition: Catalysis of the reactions: (R)-2-hydroxypropyl-CoM = H-S-CoM + (R)-1,2-epoxypropane, and (S)-2-hydroxypropyl-CoM = H-S-CoM + (S)-1,2-epoxypropane. Sources: EC:4.4.1.23 Relationships: is a type of carbon-sulfur lyase activity [GO:0016846] Also known as: (R)-2-hydroxypropyl-CoM 2-mercaptoethanesulfonate lyase (cyclizing; epoxyalkane-ring-forming), (R)-[or (S)-]2-hydroxypropyl-CoM:2-mercaptoethanesulfonate lyase (epoxyalkane-ring-forming), 2-hydroxypropyl-CoM:2-mercaptoethanesulfonate lyase (epoxyalkane-ring-forming), EaCoMT activity, coenzyme M-epoxyalkane ligase activity, epoxyalkane:2-mercaptoethanesulfonate transferase activity, epoxyalkane:CoM transferase activity, epoxyalkane:coenzyme M transferase activity, epoxyalkyl:CoM transferase activity, epoxypropane:coenzyme M transferase activity, epoxypropyl:CoM transferase activity